{
  "term_id": "UNKNOWN:0001",
  "gene_name": "Zinc finger CCCH domain-containing protein 13",
  "gene": "UniProtKB:Q5T200",
  "gene_symbol": "ZC3H13",
  "term_label": "Unknown molecular function"
}